{
  "gene_symbol": "TRMT1",
  "term_id": "GO:0005634",
  "gene": "UniProtKB:Q9NXH9",
  "gene_name": "tRNA (guanine(26)-N(2))-dimethyltransferase",
  "term_label": "nucleus"
}